{
  "gene_name": "DNA-directed RNA polymerase II subunit RPB1",
  "term_id": "UNKNOWN:0001",
  "gene_symbol": "POLR2A",
  "gene": "UniProtKB:P24928",
  "term_label": "Unknown molecular function"
}